{
  "gene_symbol": "MTA1",
  "term_label": "histone deacetylase binding",
  "term_id": "GO:0042826",
  "gene_name": "Metastasis-associated protein MTA1",
  "gene": "UniProtKB:Q13330"
}